negative regulation of bile acid biosynthetic process [GO:0070858] (biological process) Sources: GOC:BHF, GOC:mah Relationships: is a type of GO:0010894; is a type of negative regulation of small molecule metabolic process [GO:0062014]; is a type of regulation of bile acid biosynthetic process [GO:0070857]; negatively regulates GO:0006699 Also known as: down regulation of bile acid biosynthetic process, down-regulation of bile acid biosynthetic process, downregulation of bile acid biosynthetic process, negative regulation of bile acid anabolism, negative regulation of bile acid biosynthesis, negative regulation of bile acid formation, negative regulation of bile acid synthesis, inhibition of bile acid biosynthetic process Definition: Any process that stops, prevents, or reduces the frequency, rate or extent of the chemical reactions and pathways resulting in the formation of bile acids.